{
  "term_label": "external side of plasma membrane",
  "gene_name": "C-type lectin domain family 4 member K",
  "term_id": "GO:0009897",
  "gene_symbol": "CD207",
  "gene": "UniProtKB:Q9UJ71"
}